{
  "term_id": "GO:0016477",
  "term_label": "cell migration",
  "gene_symbol": "PAK2",
  "gene": "UniProtKB:Q13177",
  "gene_name": "Serine_threonine-protein kinase PAK 2"
}